{
  "term_id": "GO:0005886",
  "gene_name": "Transmembrane protein 233",
  "gene_symbol": "TMEM233",
  "term_label": "plasma membrane",
  "gene": "UniProtKB:B4DJY2"
}